{
  "term_id": "UNKNOWN:0002",
  "gene": "UniProtKB:Q86UU5",
  "gene_name": "Gametogenetin",
  "term_label": "Unknown biological process",
  "gene_symbol": "GGN"
}